1,3-alpha-L-fucosidase activity [GO:0033932] (molecular function) Relationships: is a type of GO:0004560 Sources: EC:3.2.1.111 Also known as: 3-alpha-L-fucosyl-N-acetylglucosaminyl-glycoprotein fucohydrolase activity, almond emulsin fucosidase I activity Definition: Catalysis of the hydrolysis of (1->3) linkages between alpha-L-fucose and N-acetylglucosamine residues in glycoproteins.